{
  "term_label": "ferrous iron transmembrane transporter activity",
  "term_id": "GO:0015093",
  "gene_symbol": "SLC25A28",
  "gene": "UniProtKB:Q96A46",
  "gene_name": "Mitoferrin-2"
}